{
  "gene": "UniProtKB:P19801",
  "term_id": "GO:0005507",
  "gene_name": "Amiloride-sensitive amine oxidase [copper-containing]",
  "term_label": "copper ion binding",
  "gene_symbol": "AOC1"
}